{
  "gene_name": "IQ motif and SEC7 domain-containing protein 3",
  "gene": "UniProtKB:Q9UPP2",
  "term_label": "guanyl-nucleotide exchange factor activity",
  "gene_symbol": "IQSEC3",
  "term_id": "GO:0005085"
}